{
  "term_label": "Unknown biological process",
  "gene_name": "Leydig cell tumor 10 kDa protein homolog",
  "term_id": "UNKNOWN:0002",
  "gene_symbol": "C19orf53",
  "gene": "UniProtKB:Q9UNZ5"
}